{
  "gene": "UniProtKB:Q9NSQ0",
  "gene_name": "Putative ribosomal RNA-processing protein 7 homolog B",
  "gene_symbol": "RRP7BP",
  "term_label": "UTP-C complex",
  "term_id": "GO:0034456"
}